{
  "term_id": "GO:0006357",
  "gene": "UniProtKB:P17097",
  "gene_name": "Zinc finger protein 7",
  "gene_symbol": "ZNF7",
  "term_label": "regulation of transcription by RNA polymerase II"
}